{
  "gene_symbol": "PISD",
  "gene": "UniProtKB:Q9UG56",
  "term_id": "GO:0004609",
  "term_label": "phosphatidylserine decarboxylase activity",
  "gene_name": "Phosphatidylserine decarboxylase proenzyme, mitochondrial"
}